positive regulation of calcitonin secretion [GO:1904364] (biological process) Definition: Any process that activates or increases the frequency, rate or extent of calcitonin secretion. References: PMID:11278900 Sources: GOC:TermGenie, GO_REF:0000058 Also known as: up regulation of calcitonin secretion, up-regulation of calcitonin secretion, upregulation of calcitonin secretion, activation of calcitonin secretion Relationships: is a type of GO:0090277; is a type of regulation of calcitonin secretion [GO:1904362]; positively regulates calcitonin secretion [GO:0036161]